rhamnose catabolic process [GO:0019301] (biological process) Regulation: regulated by regulation of rhamnose catabolic process [GO:0043463] Subtypes: anaerobic rhamnose catabolic process [GO:0019304] Also known as: rhamnose breakdown, rhamnose catabolism, rhamnose degradation Relationships: is a type of GO:0019320 Definition: The chemical reactions and pathways resulting in the breakdown of rhamnose, the hexose 6-deoxy-L-mannose. Sources: ISBN:0198506732